{
  "term_id": "GO:0001508",
  "gene": "UniProtKB:O95837",
  "gene_symbol": "GNA14",
  "gene_name": "Guanine nucleotide-binding protein subunit alpha-14",
  "term_label": "action potential"
}